positive regulation of striated muscle cell differentiation [GO:0051155] (biological process) Also known as: up regulation of striated muscle cell differentiation, up-regulation of striated muscle cell differentiation, upregulation of striated muscle cell differentiation, activation of striated muscle cell differentiation, stimulation of striated muscle cell differentiation Definition: Any process that activates or increases the frequency, rate or extent of striated muscle cell differentiation. Relationships: is a type of positive regulation of muscle cell differentiation [GO:0051149]; is_a GO:0051153; RO_0002213 striated muscle cell differentiation [GO:0051146] Subtypes: positive regulation of myotube differentiation [GO:0010831], positive regulation of skeletal muscle fiber development [GO:0048743], positive regulation of sarcomere organization [GO:0060298], positive regulation of cell growth involved in cardiac muscle cell development [GO:0061051], GO:2000727 Sources: CL:0000737, GOC:ai